{
  "term_id": "GO:0005886",
  "gene": "UniProtKB:Q496H8",
  "gene_symbol": "NRN1L",
  "term_label": "plasma membrane",
  "gene_name": "Neuritin-like protein"
}